{
  "term_id": "UNKNOWN:0001",
  "term_label": "Unknown molecular function",
  "gene_symbol": "DYDC1",
  "gene": "UniProtKB:Q8WWB3",
  "gene_name": "DPY30 domain-containing protein 1"
}